{
  "term_label": "Unknown molecular function",
  "gene_symbol": "TRIP13",
  "term_id": "UNKNOWN:0001",
  "gene_name": "Pachytene checkpoint protein 2 homolog",
  "gene": "UniProtKB:Q15645"
}